{
  "term_label": "Unknown molecular function",
  "gene": "UniProtKB:Q7Z713",
  "term_id": "UNKNOWN:0001",
  "gene_name": "Ankyrin repeat domain-containing protein 37",
  "gene_symbol": "ANKRD37"
}